collagen type X trimer [GO:0005599] (cellular component) Note: Collagen X trimers have been observed to form hexagonal lattices in vitro, but in vivo they have been found in a fibril associated form (PMID:19693541). References: PMID:21421911 Relationships: is a type of GO:0098642; BFO_0000050 interstitial hexagonal collagen network [GO:0098646] Definition: A collagen homotrimer of alpha1(X) chains; type X collagen triple helices form hexagonal networks (sheets).